{
  "gene_name": "Spectrin beta chain, non-erythrocytic 1",
  "gene": "UniProtKB:Q01082",
  "term_label": "protein localization to plasma membrane",
  "term_id": "GO:0072659",
  "gene_symbol": "SPTBN1"
}